{
  "gene_name": "Fibulin-5",
  "term_label": "extracellular space",
  "gene_symbol": "FBLN5",
  "term_id": "GO:0005615",
  "gene": "UniProtKB:Q9UBX5"
}